bone marrow development [GO:0048539] (biological process) Definition: The process whose specific outcome is the progression of the bone marrow over time, from its formation to the mature structure. Relationships: is a type of tissue development [GO:0009888]; is a type of hematopoietic or lymphoid organ development [GO:0048534]; is part of GO:0060348 Sources: GOC:add, ISBN:0781735149